CXCR6 chemokine receptor binding [GO:0031725] (molecular function) Relationships: is a type of CXCR chemokine receptor binding [GO:0045236] Sources: GOC:mah, GOC:nln Definition: Binding to a CXCR6 chemokine receptor. Also known as: STRL33 receptor binding, bonzo receptor binding, CXCR6 chemokine receptor ligand